{
  "term_label": "DNA-binding transcription factor activity, RNA polymerase II-specific",
  "gene_name": "Zinc finger protein 75D",
  "term_id": "GO:0000981",
  "gene": "UniProtKB:P51815",
  "gene_symbol": "ZNF75D"
}